{
  "term_id": "GO:0005634",
  "gene_symbol": "MAGEB4",
  "term_label": "nucleus",
  "gene_name": "Melanoma-associated antigen B4",
  "gene": "UniProtKB:O15481"
}